{
  "term_id": "GO:0005789",
  "term_label": "endoplasmic reticulum membrane",
  "gene": "UniProtKB:P00167",
  "gene_name": "Cytochrome b5",
  "gene_symbol": "CYB5A"
}